{
  "term_label": "cell differentiation",
  "term_id": "GO:0030154",
  "gene_name": "NK1 transcription factor-related protein 2",
  "gene": "UniProtKB:Q9UD57",
  "gene_symbol": "NKX1-2"
}